UUG codon-amino acid adaptor activity [GO:0033404] (molecular function) Also known as: TTG codon-amino acid adaptor activity, leucine tRNA Definition: A triplet codon-amino acid adaptor activity that recognizes a UUG codon. Sources: GOC:mah Note: Note that in the standard genetic code, TTG codes for leucine. Relationships: is a type of triplet codon-amino acid adaptor activity [GO:0030533]